{
  "term_id": "GO:0005874",
  "term_label": "microtubule",
  "gene_name": "Kinesin-like protein KIF1B",
  "gene_symbol": "KIF1B",
  "gene": "UniProtKB:O60333"
}